regulation of matrix metallopeptidase secretion [GO:1904464] (biological process) Definition: Any process that modulates the frequency, rate or extent of matrix metallopeptidase secretion. Relationships: is a type of GO:0050708; regulates matrix metallopeptidase secretion [GO:1990773] References: PMID:8679543 Sources: GOC:TermGenie, GO_REF:0000058 Also known as: regulation of MMP secretion, regulation of matrix metalloproteinase secretion Subtypes: negative regulation of matrix metallopeptidase secretion [GO:1904465], positive regulation of matrix metallopeptidase secretion [GO:1904466]